{
  "gene_name": "Chromodomain-helicase-DNA-binding protein 6",
  "term_id": "GO:0016887",
  "gene": "UniProtKB:Q8TD26",
  "gene_symbol": "CHD6",
  "term_label": "ATP hydrolysis activity"
}